{
  "term_id": "GO:0043596",
  "gene": "UniProtKB:Q6ZRQ5",
  "gene_name": "Protein MMS22-like",
  "term_label": "nuclear replication fork",
  "gene_symbol": "MMS22L"
}